immunoglobulin mediated immune response [GO:0016064] (biological process) Definition: An immune response mediated by immunoglobulins, whether cell-bound or in solution. Sources: GOC:add, GO_REF:0000022, ISBN:0781735149 Also known as: antibody-mediated immune response Relationships: is a type of B cell mediated immunity [GO:0019724] Subtypes: GO:0001802, type II hypersensitivity [GO:0002445], humoral immune response mediated by circulating immunoglobulin [GO:0002455], GO:0016068, GO:0097281, immunoglobulin-mediated neutralization [GO:0097282] Regulation: regulated by GO:0002889; negatively regulated by GO:0002890; RO_0002213 by positive regulation of immunoglobulin mediated immune response [GO:0002891]